regulation of transmembrane receptor protein serine/threonine kinase signaling pathway [GO:0090092] (biological process) Subtypes: regulation of transforming growth factor beta receptor signaling pathway [GO:0017015], regulation of BMP signaling pathway [GO:0030510], GO:0032925, GO:0090100, negative regulation of transmembrane receptor protein serine/threonine kinase signaling pathway [GO:0090101], regulation of anti-Mullerian hormone signaling pathway [GO:1902612] Sources: GOC:dph, GOC:tb Relationships: is a type of regulation of signal transduction [GO:0009966]; regulates cell surface receptor protein serine/threonine kinase signaling pathway [GO:0007178] Definition: Any process that modulates the rate, frequency, or extent of the series of molecular signals generated as a consequence of a transmembrane receptor serine/threonine kinase binding to its physiological ligand. Also known as: regulation of transmembrane receptor protein serine/threonine kinase signalling pathway